{
  "gene_symbol": "IFNL1",
  "term_label": "defense response to virus",
  "gene_name": "Interferon lambda-1",
  "gene": "UniProtKB:Q8IU54",
  "term_id": "GO:0051607"
}